{
  "gene": "UniProtKB:O15519",
  "gene_name": "CASP8 and FADD-like apoptosis regulator",
  "gene_symbol": "CFLAR",
  "term_label": "extrinsic apoptotic signaling pathway via death domain receptors",
  "term_id": "GO:0008625"
}